{
  "gene": "UniProtKB:A0A1B0GUA9",
  "gene_name": "Uncharacterized protein C13orf46",
  "term_id": "UNKNOWN:0002",
  "term_label": "Unknown biological process",
  "gene_symbol": "C13orf46"
}